carbon catabolite activation of transcription from RNA polymerase II promoter [GO:0000436] (BP) Definition: Any process involving carbon catabolites that activates or increases the frequency, rate or extent of transcription from an RNA polymerase II promoter. Subtypes: positive regulation of transcription from RNA polymerase II promoter by glucose [GO:0000432], GO:0000435, GO:0061414, GO:0061429 Relationships: is a type of carbon catabolite regulation of transcription from RNA polymerase II promoter [GO:0000429]; is a type of positive regulation of transcription by RNA polymerase II [GO:0045944]; is a type of GO:0045991 Sources: GOC:krc Also known as: positive regulation of transcription from RNA polymerase II promoter by carbon catabolites